{
  "term_label": "protein import into peroxisome membrane",
  "gene": "UniProtKB:P40855",
  "gene_symbol": "PEX19",
  "term_id": "GO:0045046",
  "gene_name": "Peroxisomal biogenesis factor 19"
}